{
  "gene": "UniProtKB:P80098",
  "term_label": "antimicrobial humoral immune response mediated by antimicrobial peptide",
  "term_id": "GO:0061844",
  "gene_symbol": "CCL7",
  "gene_name": "C-C motif chemokine 7"
}